{
  "gene": "UniProtKB:Q8IV01",
  "gene_name": "Synaptotagmin-12",
  "gene_symbol": "SYT12",
  "term_id": "GO:0005544",
  "term_label": "calcium-dependent phospholipid binding"
}